{
  "term_label": "ketone body biosynthetic process",
  "gene": "UniProtKB:Q8TB92",
  "gene_name": "3-hydroxy-3-methylglutaryl-CoA lyase, cytoplasmic",
  "term_id": "GO:0046951",
  "gene_symbol": "HMGCLL1"
}